positive regulation of transforming growth factor beta3 production [GO:0032916] (biological process) Sources: GOC:mah Relationships: is a type of regulation of transforming growth factor beta3 production [GO:0032910]; is_a GO:0071636; positively regulates transforming growth factor beta3 production [GO:0032907] Also known as: positive regulation of TGF-B3 production, positive regulation of TGFB3 production, positive regulation of transforming growth factor-beta3 production, up regulation of transforming growth factor-beta3 production, up-regulation of transforming growth factor-beta3 production, upregulation of transforming growth factor-beta3 production, activation of transforming growth factor-beta3 production, stimulation of transforming growth factor-beta3 production Definition: Any process that activates or increases the frequency, rate, or extent of production of transforming growth factor-beta3.